3-isopropylmalate dehydratase activity [GO:0003861] (molecular function) Relationships: is a type of hydro-lyase activity [GO:0016836] Also known as: (2R,3S)-3-isopropylmalate hydro-lyase (2-isopropylmaleate-forming), (2R,3S)-3-isopropylmalate hydro-lyase activity, alpha-IPM isomerase activity, alpha-isopropylmalate isomerase activity, beta-isopropylmalate dehydratase activity, isopropylmalate isomerase activity Definition: Catalysis of the reaction: (2R,3S)-3-isopropylmalate = (2S)-2-isopropylmalate. Sources: EC:4.2.1.33